negative regulation of protein localization to cell division site involved in mitotic actomyosin contractile ring assembly [GO:0110084] (biological process) References: PMID:29343550 Sources: GOC:vw Definition: Any process that stops, prevents, or reduces the frequency, rate or extent of protein localization to cell division site involved in mitotic actomyosin contractile ring assembly. Relationships: is a type of GO:0110082; is a type of negative regulation of mitotic actomyosin contractile ring assembly [GO:1903500]; is a type of negative regulation of protein localization [GO:1903828]; negatively regulates protein localization to cell division site involved in mitotic actomyosin contractile ring assembly [GO:1903476]